{
  "term_id": "GO:0005739",
  "gene_name": "Mitochondrial ubiquitin ligase activator of NFKB 1",
  "term_label": "mitochondrion",
  "gene": "UniProtKB:Q969V5",
  "gene_symbol": "MUL1"
}